{
  "gene": "UniProtKB:P59665",
  "gene_symbol": "DEFA1B",
  "term_id": "GO:0061844",
  "gene_name": "Neutrophil defensin 1",
  "term_label": "antimicrobial humoral immune response mediated by antimicrobial peptide"
}